{
  "term_id": "GO:0008083",
  "gene_name": "Neurotrophin-4",
  "gene_symbol": "NTF4",
  "term_label": "growth factor activity",
  "gene": "UniProtKB:P34130"
}